{
  "gene_symbol": "PFKL",
  "gene_name": "ATP-dependent 6-phosphofructokinase, liver type",
  "gene": "UniProtKB:P17858",
  "term_id": "GO:0006002",
  "term_label": "fructose 6-phosphate metabolic process"
}